{
  "gene": "UniProtKB:Q9NT99",
  "term_label": "glutamatergic synapse",
  "term_id": "GO:0098978",
  "gene_name": "Leucine-rich repeat-containing protein 4B",
  "gene_symbol": "LRRC4B"
}